epithelial cell-cell adhesion [GO:0090136] (biological process) Subtypes: follicle cell of egg chamber-cell adhesion [GO:0007299], endothelial cell-cell adhesion [GO:0071603], epithelial cell-cell adhesion involved in epithelium migration [GO:0090137], melanocyte adhesion [GO:0097326] Sources: GOC:ascb_2009, GOC:dph, GOC:tb Definition: The attachment of an epithelial cell to another epithelial cell via adhesion molecules. Relationships: is a type of cell-cell adhesion [GO:0098609]